sarcoplasmic reticulum membrane [GO:0033017] (cellular component) Sources: GOC:rph Subtypes: junctional sarcoplasmic reticulum membrane [GO:0014701], free sarcoplasmic reticulum membrane [GO:0014702] Definition: The lipid bilayer surrounding the sarcoplasmic reticulum. Relationships: is a type of endoplasmic reticulum membrane [GO:0005789]; is a type of GO:0098588; is part of sarcoplasmic reticulum [GO:0016529]